21U-RNA metabolic process [GO:0034585] (biological process) Subtypes: 21U-RNA catabolic process [GO:0034586] Also known as: 21U-RNA metabolism Definition: The chemical reactions and pathways involving 21U-RNAs, a class of single-stranded RNA molecules of about 21 nucleotides in length characterized by a uridine 5'-monophosphate and a modified 3' end resistant to periodate degradation. 21U-RNAs are derived from distinct, autonomously expressed loci within the genome. Sources: GOC:kmv Relationships: is a type of RNA metabolic process [GO:0016070]